methanogenesis, from acetate [GO:0019385] (BP) Sources: GOC:ai Relationships: is a type of GO:0006083; is_a methanogenesis [GO:0015948] Definition: The formation of methane, a colorless, odorless, flammable gas with the formula CH4, from other components, including acetate. Also known as: methane biosynthesis from acetate, methane biosynthetic process from acetate